regulation of translation at presynapse [GO:0140244] (biological process) Note: Note that this term was created for the SynGO project, and will be obsoleted when the SynGO annotations are made in Noctua. Subtypes: GO:0099577 Definition: Any process that regulates translation occurring at the presynapse. References: PMID:20427644 Relationships: is_a regulation of translation at synapse [GO:0140243]; occurs in presynapse [GO:0098793]